{
  "gene_symbol": "C4orf3",
  "gene": "UniProtKB:Q8WVX3",
  "term_label": "Unknown cellular component",
  "gene_name": "Uncharacterized protein C4orf3",
  "term_id": "UNKNOWN:0003"
}